{
  "gene_name": "Cytosolic carboxypeptidase 2",
  "term_label": "tubulin binding",
  "gene": "UniProtKB:Q5U5Z8",
  "term_id": "GO:0015631",
  "gene_symbol": "AGBL2"
}